{
  "gene_name": "Zinc finger protein ZFPM2",
  "gene": "UniProtKB:Q8WW38",
  "term_label": "positive regulation of transcription by RNA polymerase II",
  "term_id": "GO:0045944",
  "gene_symbol": "ZFPM2"
}